SOS response [GO:0009432] (biological process) Relationships: is_a DNA damage response [GO:0006974] References: PMID:16000023 Sources: GOC:jl Definition: An error-prone process for repairing damaged microbial DNA.